DNA double-strand break processing involved in repair via synthesis-dependent strand annealing [GO:0010791] (biological process) Relationships: is a type of DNA double-strand break processing [GO:0000729]; BFO_0000050 double-strand break repair via synthesis-dependent strand annealing [GO:0045003] Sources: GOC:dph, GOC:tb Definition: The 5' to 3' exonucleolytic resection of the DNA at the site of the break to form a 3' single-strand DNA overhang that results in the repair of a double strand break via synthesis-dependent strand annealing.